{
  "term_label": "Unknown biological process",
  "gene_symbol": "APOL4",
  "term_id": "UNKNOWN:0002",
  "gene": "UniProtKB:Q9BPW4",
  "gene_name": "Apolipoprotein L4"
}